{
  "gene": "UniProtKB:P61960",
  "gene_symbol": "UFM1",
  "term_id": "GO:0034976",
  "term_label": "response to endoplasmic reticulum stress",
  "gene_name": "Ubiquitin-fold modifier 1"
}